{
  "gene_symbol": "SLC35F5",
  "gene_name": "Solute carrier family 35 member F5",
  "term_label": "Unknown biological process",
  "gene": "UniProtKB:Q8WV83",
  "term_id": "UNKNOWN:0002"
}